{
  "term_id": "GO:0007265",
  "gene_symbol": "RAPGEF2",
  "gene": "UniProtKB:Q9Y4G8",
  "term_label": "Ras protein signal transduction",
  "gene_name": "Rap guanine nucleotide exchange factor 2"
}